{
  "gene_symbol": "RBPJ",
  "gene": "UniProtKB:Q06330",
  "term_id": "GO:0000981",
  "gene_name": "Recombining binding protein suppressor of hairless",
  "term_label": "DNA-binding transcription factor activity, RNA polymerase II-specific"
}